{
  "gene_name": "Serine_threonine_tyrosine-interacting-like protein 2",
  "gene": "UniProtKB:Q5VZP5",
  "term_label": "MAP kinase phosphatase activity",
  "gene_symbol": "STYXL2",
  "term_id": "GO:0033549"
}